{
  "gene_name": "PDZ and LIM domain protein 2",
  "gene_symbol": "PDLIM2",
  "term_label": "filamentous actin",
  "term_id": "GO:0031941",
  "gene": "UniProtKB:Q96JY6"
}